{
  "gene": "UniProtKB:Q9Y5H4",
  "gene_name": "Protocadherin gamma-A1",
  "term_id": "GO:0005886",
  "term_label": "plasma membrane",
  "gene_symbol": "PCDHGA1"
}